{
  "gene": "UniProtKB:Q96SM3",
  "gene_name": "Probable carboxypeptidase X1",
  "gene_symbol": "CPXM1",
  "term_id": "UNKNOWN:0001",
  "term_label": "Unknown molecular function"
}